{
  "gene_symbol": "DGKI",
  "term_label": "intracellular signal transduction",
  "gene": "UniProtKB:O75912",
  "term_id": "GO:0035556",
  "gene_name": "Diacylglycerol kinase iota"
}